negative regulation of fibroblast chemotaxis [GO:1905211] (biological process) Relationships: is a type of GO:0030336; is a type of negative regulation of chemotaxis [GO:0050922]; is_a GO:1905210; negatively regulates fibroblast chemotaxis [GO:1990956] References: PMID:8760137 Sources: GOC:TermGenie, GO_REF:0000058 Definition: Any process that stops, prevents or reduces the frequency, rate or extent of fibroblast chemotaxis. Also known as: down regulation of fibroblast chemotaxis, down-regulation of fibroblast chemotaxis, downregulation of fibroblast chemotaxis, inhibition of fibroblast chemotaxis